{
  "gene": "UniProtKB:Q5PT55",
  "term_label": "bile acid:sodium symporter activity",
  "term_id": "GO:0008508",
  "gene_symbol": "SLC10A5",
  "gene_name": "Sodium_bile acid cotransporter 5"
}